negative regulation of ERK1 and ERK2 cascade [GO:0070373] (biological process) Definition: Any process that stops, prevents, or reduces the frequency, rate or extent of signal transduction mediated by the ERK1 and ERK2 cascade. Relationships: is a type of negative regulation of MAPK cascade [GO:0043409]; is a type of regulation of ERK1 and ERK2 cascade [GO:0070372]; negatively regulates ERK1 and ERK2 cascade [GO:0070371] Also known as: negative regulation of ERK cascade, down regulation of ERK1 and ERK2 cascade, down-regulation of ERK1 and ERK2 cascade, downregulation of ERK1 and ERK2 cascade, negative regulation of ERK1 and ERK2 signaling pathway, negative regulation of ERK1 and ERK2 signalling pathway, negative regulation of ERK1/2 cascade, inhibition of ERK1 and ERK2 cascade, negative regulation of ERK1 cascade, negative regulation of ERK2 cascade, negative regulation of MAPK1 cascade, negative regulation of MAPK3 cascade Sources: GOC:add, ISBN:0121245462, ISBN:0896039986